{
  "gene_name": "Pregnancy-specific beta-1-glycoprotein 11",
  "gene_symbol": "PSG11",
  "term_label": "plasma membrane",
  "gene": "UniProtKB:Q9UQ72",
  "term_id": "GO:0005886"
}